{
  "term_label": "muscle organ development",
  "term_id": "GO:0007517",
  "gene_name": "Homeobox protein Mohawk",
  "gene": "UniProtKB:Q8IYA7",
  "gene_symbol": "MKX"
}